L-glutamate gamma-semialdehyde dehydrogenase activity [GO:0003842] (MF) Also known as: 1-pyrroline dehydrogenase, 1-pyrroline-5-carboxylate dehydrogenase activity, 1-pyrroline-5-carboxylate:NAD+ oxidoreductase activity, L-pyrroline-5-carboxylate-NAD+ oxidoreductase activity, delta1-pyrroline-5-carboxylate dehydrogenase activity, pyrroline-5-carboxylate dehydrogenase activity, pyrroline-5-carboxylic acid dehydrogenase activity Sources: RHEA:30235 Definition: L-glutamate 5-semialdehyde + NAD+ + H2O = L-glutamate + NADH + 2 H+. Note: (S)-1-pyrroline-5-carboxylate is in spontaneous equilibrium with its tautomer L-glutamate gamma-semialdehyde. The activity can also oxidize other 1-pyrrolines, e.g. oxidation of 3-hydroxy-1-pyrroline-5-carboxylate to 4-hydroxyglutamate, and oxidation of (R)-1-pyrroline-5-carboxylate to D-glutamate. Relationships: is a type of GO:0016620